{
  "gene_symbol": "Q5BKY6",
  "term_id": "UNKNOWN:0003",
  "term_label": "Unknown cellular component",
  "gene": "UniProtKB:Q5BKY6",
  "gene_name": "Putative uncharacterized protein DKFZp434K191"
}